galactosyltransferase activity [GO:0008378] (molecular function) Sources: ISBN:0198506732 Relationships: is a type of hexosyltransferase activity [GO:0016758] Subtypes: alpha-1,3-galactosyltransferase activity [GO:0001962], alpha-1,2-galactosyltransferase activity [GO:0031278], UDP-galactosyltransferase activity [GO:0035250], galactolipid galactosyltransferase activity [GO:0046480], raffinose-raffinose alpha-galactotransferase activity [GO:0047234], galactinol-raffinose galactosyltransferase activity [GO:0047268], GO:0047274, beta-1,3-galactosyltransferase activity [GO:0048531], hydroxyproline O-galactosyltransferase activity [GO:1990714] Definition: Catalysis of the transfer of a galactosyl group to an acceptor molecule, typically another carbohydrate or a lipid.